positive regulation of emericellin biosynthetic process [GO:1900836] (biological process) Sources: GOC:TermGenie, GOC:di Relationships: is a type of GO:1900185; is a type of GO:1900378; is a type of regulation of emericellin biosynthetic process [GO:1900834]; positively regulates emericellin biosynthetic process [GO:1900766] Definition: Any process that activates or increases the frequency, rate or extent of emericellin biosynthetic process.